{
  "gene_name": "Long-chain specific acyl-CoA dehydrogenase, mitochondrial",
  "term_id": "GO:0019254",
  "term_label": "carnitine metabolic process, CoA-linked",
  "gene": "UniProtKB:P28330",
  "gene_symbol": "ACADL"
}